cell-cell adhesion involved in sealing an epithelial fold [GO:0060607] (BP) Sources: GOC:dph Relationships: is a type of cell-cell adhesion [GO:0098609]; is part of tube closure [GO:0060606] Definition: The attachment of one cell to another cell along the edges of two epithelial folds, giving rise to the lumen of an epithelial tube. Subtypes: cell-cell adhesion involved in neural tube closure [GO:0060608]